{
  "gene": "UniProtKB:Q969G6",
  "gene_name": "Riboflavin kinase",
  "gene_symbol": "RFK",
  "term_id": "GO:0005739",
  "term_label": "mitochondrion"
}